regulation of defense response [GO:0031347] (biological process) Subtypes: regulation of antimicrobial humoral response [GO:0002759], regulation of systemic acquired resistance [GO:0010112], GO:0010185, GO:0031348, positive regulation of defense response [GO:0031349], GO:0045088, regulation of defense response to virus [GO:0050688], GO:0050727, regulation of neutrophil mediated killing of symbiont cell [GO:0070949], regulation of defense response to fungus [GO:1900150], GO:1900424, regulation of defense response to oomycetes [GO:1902288], GO:2000068, regulation of defense response by callose deposition [GO:2000071], regulation of behavioral fear response [GO:2000822] Sources: GOC:mah Definition: Any process that modulates the frequency, rate or extent of a defense response. Relationships: is_a regulation of response to stress [GO:0080134]; regulates defense response [GO:0006952]